activation-induced B cell apoptotic process [GO:0071948] (biological process) Definition: B cell apoptotic process that occurs upon engagement of either the B cell receptor or CD40. Engagement of either receptor, but not both, leads to expression of fas or related receptors that make the B cell susceptible to fas-ligand mediated death. References: PMID:11032170, PMID:19300454 Sources: GOC:mtg_apoptosis, GOC:tfm Relationships: is a type of B cell apoptotic process [GO:0001783] Also known as: AICD, activated B cell apoptosis, antigen-driven apoptosis, activation-induced B-cell apoptosis, activation-induced cell death of B cells, activation-induced cell death of B lymphocytes, activation-induced cell death of B-cells, activation-induced cell death of B-lymphocytes, activation-induced B cell apoptosis